{
  "gene_symbol": "NHLRC3",
  "gene_name": "NHL repeat-containing protein 3",
  "term_id": "UNKNOWN:0003",
  "gene": "UniProtKB:Q5JS37",
  "term_label": "Unknown cellular component"
}